{
  "term_id": "UNKNOWN:0003",
  "gene_symbol": "SPATA22",
  "term_label": "Unknown cellular component",
  "gene_name": "Spermatogenesis-associated protein 22",
  "gene": "UniProtKB:Q8NHS9"
}